{
  "gene_name": "Regulator of chromosome condensation",
  "term_id": "GO:0007346",
  "gene": "UniProtKB:P18754",
  "term_label": "regulation of mitotic cell cycle",
  "gene_symbol": "RCC1"
}